{
  "gene": "UniProtKB:Q6NUT2",
  "term_label": "spermatid development",
  "gene_symbol": "DPY19L2",
  "term_id": "GO:0007286",
  "gene_name": "Probable C-mannosyltransferase DPY19L2"
}